{
  "gene": "UniProtKB:Q32P41",
  "gene_symbol": "TRMT5",
  "term_id": "GO:0005737",
  "term_label": "cytoplasm",
  "gene_name": "tRNA (guanine(37)-N1)-methyltransferase"
}